{
  "gene": "UniProtKB:O75715",
  "term_id": "GO:0004602",
  "gene_name": "Epididymal secretory glutathione peroxidase",
  "term_label": "glutathione peroxidase activity",
  "gene_symbol": "GPX5"
}